{
  "gene_name": "Immunoglobulin heavy variable 3-53",
  "gene_symbol": "IGHV3-53",
  "term_id": "UNKNOWN:0003",
  "term_label": "Unknown cellular component",
  "gene": "UniProtKB:P01767"
}